{
  "gene_name": "Protein tweety homolog 1",
  "term_label": "Unknown biological process",
  "gene": "UniProtKB:Q9H313",
  "term_id": "UNKNOWN:0002",
  "gene_symbol": "TTYH1"
}